{
  "gene_symbol": "KRTAP12-3",
  "term_label": "Unknown molecular function",
  "gene": "UniProtKB:P60328",
  "gene_name": "Keratin-associated protein 12-3",
  "term_id": "UNKNOWN:0001"
}